{
  "term_id": "GO:0019221",
  "term_label": "cytokine-mediated signaling pathway",
  "gene_symbol": "IL23R",
  "gene_name": "Interleukin-23 receptor",
  "gene": "UniProtKB:Q5VWK5"
}